regulation of peroxisome size [GO:0044375] (biological process) Definition: Any process that modulates the volume of a peroxisome, a small, membrane-bounded organelle that uses dioxygen (O2) to oxidize organic molecules. Sources: GOC:jl Relationships: is a type of regulation of cellular component size [GO:0032535]